vitamin A biosynthetic process [GO:0035238] (biological process) Definition: The chemical reactions and pathways resulting in the formation of any of the vitamin A compounds, retinol, retinal (retinaldehyde) and retinoic acid. Animals cannot synthesize vitamin A de novo, but form it through oxidative cleavage of carotenoids. References: PMID:11158606 Also known as: vitamin A anabolism, vitamin A biosynthesis, vitamin A formation, vitamin A synthesis Relationships: is a type of vitamin A metabolic process [GO:0006776]; is a type of GO:0016102; is a type of fat-soluble vitamin biosynthetic process [GO:0042362]